{
  "term_id": "UNKNOWN:0001",
  "gene_symbol": "SIRPB2",
  "gene_name": "Signal-regulatory protein beta-2",
  "term_label": "Unknown molecular function",
  "gene": "UniProtKB:Q5JXA9"
}